neuroblast division [GO:0055057] (biological process) Also known as: neuroblast cell division Subtypes: neuroblast division in subpallium [GO:0021848], neuroblast division in subventricular zone [GO:0021849], forebrain neuroblast division [GO:0021873], symmetric neuroblast division [GO:0055058], asymmetric neuroblast division [GO:0055059] Relationships: is a type of cell division [GO:0051301]; is part of neuroblast proliferation [GO:0007405] References: PMID:11163136, PMID:11250167 Definition: The process resulting in the physical partitioning and separation of a neuroblast into daughter cells. A neuroblast is any cell that will divide and give rise to a neuron.